{
  "term_label": "cytosol",
  "term_id": "GO:0005829",
  "gene": "UniProtKB:O95429",
  "gene_symbol": "BAG4",
  "gene_name": "BAG family molecular chaperone regulator 4"
}